{
  "gene": "UniProtKB:P36402",
  "term_id": "GO:1990907",
  "term_label": "beta-catenin-TCF complex",
  "gene_name": "Transcription factor 7",
  "gene_symbol": "TCF7"
}